histone H2B ubiquitin ligase activity [GO:0141054] (molecular function) Definition: Catalysis of the transfer of ubiquitin to a histone H2B substrate. Subtypes: histone H2B C-terminal K residue ubiquitin ligase activity [GO:0140850] Relationships: is a type of histone ubiquitin ligase activity [GO:0140852] References: PMID:25303536